cell proliferation involved in mesonephros development [GO:0061209] (biological process) Sources: GOC:mtg_kidney_jan10 Subtypes: mesonephric mesenchymal cell proliferation involved in mesonephros development [GO:0061222], GO:0061225, mesonephric glomerular mesangial cell proliferation involved in mesonephros development [GO:0061269], mesenchymal cell proliferation involved in ureteric bud development [GO:0072138] Relationships: is a type of cell proliferation involved in kidney development [GO:0072111]; is part of mesonephros development [GO:0001823] Definition: The multiplication or reproduction of cells, resulting in the expansion of the population in the mesonephros. Regulation: regulated by regulation of cell proliferation involved in mesonephros development [GO:2000606]; negatively regulated by negative regulation of cell proliferation involved in mesonephros development [GO:2000607]; positively regulated by positive regulation of cell proliferation involved in mesonephros development [GO:2000608]